{
  "term_id": "GO:0006357",
  "gene": "UniProtKB:Q9H7R5",
  "gene_symbol": "ZNF665",
  "gene_name": "Zinc finger protein 665",
  "term_label": "regulation of transcription by RNA polymerase II"
}